{
  "gene_symbol": "SLC26A11",
  "term_label": "chloride transmembrane transport",
  "gene": "UniProtKB:Q86WA9",
  "gene_name": "Sodium-independent sulfate anion transporter",
  "term_id": "GO:1902476"
}